{
  "gene_symbol": "RELL1",
  "gene": "UniProtKB:Q8IUW5",
  "term_label": "positive regulation of p38MAPK cascade",
  "term_id": "GO:1900745",
  "gene_name": "RELT-like protein 1"
}